nicotinate transmembrane transporter activity [GO:0090416] (molecular function) Relationships: is a type of monocarboxylic acid transmembrane transporter activity [GO:0008028]; is part of GO:2001142 Sources: GOC:tb Definition: Enables the transfer of nicotinate from one side of a membrane to the other.